{
  "gene_symbol": "UBE2D1",
  "term_label": "protein K48-linked ubiquitination",
  "gene_name": "Ubiquitin-conjugating enzyme E2 D1",
  "term_id": "GO:0070936",
  "gene": "UniProtKB:P51668"
}